{
  "term_id": "GO:0005634",
  "term_label": "nucleus",
  "gene_symbol": "EHMT1",
  "gene_name": "Histone-lysine N-methyltransferase EHMT1",
  "gene": "UniProtKB:Q9H9B1"
}